{
  "term_id": "GO:0035999",
  "gene": "UniProtKB:P42898",
  "term_label": "tetrahydrofolate interconversion",
  "gene_symbol": "MTHFR",
  "gene_name": "Methylenetetrahydrofolate reductase (NADPH)"
}